fatty acid binding [GO:0005504] (molecular function) Definition: Binding to a fatty acid, an aliphatic monocarboxylic acids liberated from naturally occurring fats and oils by hydrolysis. Subtypes: GO:0031405, long-chain fatty acid binding [GO:0036041], leptomycin B binding [GO:1901707], GO:1904767 Sources: ISBN:0198506732 Relationships: is a type of lipid binding [GO:0008289]; is a type of GO:0033293